{
  "term_label": "response to hormone",
  "gene": "UniProtKB:P01033",
  "term_id": "GO:0009725",
  "gene_name": "Metalloproteinase inhibitor 1",
  "gene_symbol": "TIMP1"
}